{
  "term_label": "Unknown biological process",
  "gene_name": "Uncharacterized protein C13orf42",
  "term_id": "UNKNOWN:0002",
  "gene": "UniProtKB:A0A1B0GVH6",
  "gene_symbol": "C13orf42"
}